{
  "gene_symbol": "CFAP47",
  "term_label": "cilium",
  "term_id": "GO:0005929",
  "gene": "UniProtKB:Q6ZTR5",
  "gene_name": "Cilia- and flagella-associated protein 47"
}